{
  "term_label": "innate immune response",
  "gene_name": "Pyrin domain-containing protein 1",
  "term_id": "GO:0045087",
  "gene_symbol": "PYDC1",
  "gene": "UniProtKB:Q8WXC3"
}